{
  "gene_symbol": "AXIN2",
  "gene_name": "Axin-2",
  "term_label": "cell development",
  "term_id": "GO:0048468",
  "gene": "UniProtKB:Q9Y2T1"
}